{
  "gene_name": "Serine_threonine_tyrosine-interacting-like protein 1",
  "gene": "UniProtKB:Q9Y6J8",
  "term_id": "GO:0019903",
  "gene_symbol": "STYXL1",
  "term_label": "protein phosphatase binding"
}